DNA polymerase III, clamp loader chi/psi subcomplex [GO:0043847] (cellular component) Also known as: DNA polymerase III, DnaX complex, chi/psi subcomplex Relationships: is a type of nuclear protein-containing complex [GO:0140513]; is part of GO:0043846 Definition: A dimer composed of the chi and psi subunits which is a subassembly of the DNA polymerase III clamp loader complex and serves as a bridge between the DnaX complex and the single-stranded DNA-binding protein (SSB). References: PMID:12940977